{
  "gene": "UniProtKB:A0A804HJP8",
  "gene_symbol": "A0A804HJP8",
  "term_id": "UNKNOWN:0001",
  "term_label": "Unknown molecular function",
  "gene_name": "Uncharacterized protein"
}